{
  "gene_name": "Pantothenate kinase 2, mitochondrial",
  "term_label": "cytosol",
  "term_id": "GO:0005829",
  "gene_symbol": "PANK2",
  "gene": "UniProtKB:Q9BZ23"
}